{
  "gene_name": "Zinc finger C3HC-type protein 1",
  "term_id": "UNKNOWN:0001",
  "term_label": "Unknown molecular function",
  "gene": "UniProtKB:Q86WB0",
  "gene_symbol": "ZC3HC1"
}